{
  "gene": "UniProtKB:Q96JJ7",
  "gene_symbol": "TMX3",
  "term_id": "UNKNOWN:0001",
  "gene_name": "Protein disulfide-isomerase TMX3",
  "term_label": "Unknown molecular function"
}